{
  "gene_name": "Leucine-rich repeat and immunoglobulin-like domain-containing nogo receptor-interacting protein 3",
  "gene_symbol": "LINGO3",
  "gene": "UniProtKB:P0C6S8",
  "term_label": "plasma membrane",
  "term_id": "GO:0005886"
}